{
  "gene_symbol": "EBNA1BP2",
  "gene": "UniProtKB:Q99848",
  "gene_name": "Probable rRNA-processing protein EBP2",
  "term_label": "nucleolus",
  "term_id": "GO:0005730"
}